{
  "gene_symbol": "MAGEA12",
  "gene": "UniProtKB:P43365",
  "term_label": "histone deacetylase binding",
  "gene_name": "Melanoma-associated antigen 12",
  "term_id": "GO:0042826"
}